beta-alanine biosynthetic process via 3-ureidopropionate [GO:0033396] (biological process) Also known as: beta-alanine anabolism via 3-ureidopropionate, beta-alanine formation via 3-ureidopropionate, beta-alanine synthesis via 3-ureidopropionate Sources: GOC:mah, MetaCyc:PWY-3982 Relationships: is a type of GO:0019483 Definition: The chemical reactions and pathways resulting in the formation of beta-alanine via the intermediate 3-ureidopropionate.